{
  "term_id": "UNKNOWN:0002",
  "gene_symbol": "SYCE1",
  "gene": "UniProtKB:Q8N0S2",
  "term_label": "Unknown biological process",
  "gene_name": "Synaptonemal complex central element protein 1"
}